{
  "term_id": "GO:0071375",
  "gene_name": "Cytochrome P450 11B2, mitochondrial",
  "gene": "UniProtKB:P19099",
  "term_label": "cellular response to peptide hormone stimulus",
  "gene_symbol": "CYP11B2"
}